urinary tract smooth muscle contraction [GO:0014848] (biological process) Subtypes: GO:0014832, ureter smooth muscle contraction [GO:0014849] Definition: A process in which force is generated within smooth muscle tissue, resulting in a change in muscle geometry. This process occurs in the urinary tract. Force generation involves a chemo-mechanical energy conversion step that is carried out by the actin/myosin complex activity, which generates force through ATP hydrolysis. The urinary tract consists of organs of the body that produce and discharge urine. These include the kidneys, ureters, bladder, and urethra. Relationships: is a type of GO:0006939 Sources: GOC:ef, GOC:mtg_muscle, MA:0000325, MSH:D014551